{
  "gene_name": "Rho guanine nucleotide exchange factor 4",
  "term_label": "Unknown cellular component",
  "term_id": "UNKNOWN:0003",
  "gene_symbol": "ARHGEF4",
  "gene": "UniProtKB:Q9NR80"
}